{
  "term_id": "GO:0007507",
  "term_label": "heart development",
  "gene_symbol": "POPDC2",
  "gene_name": "Popeye domain-containing protein 2",
  "gene": "UniProtKB:Q9HBU9"
}